{
  "gene_name": "Ubiquitin-like modifier-activating enzyme 1",
  "gene_symbol": "UBA1",
  "term_id": "GO:0006511",
  "gene": "UniProtKB:P22314",
  "term_label": "ubiquitin-dependent protein catabolic process"
}